{
  "term_id": "GO:0001609",
  "gene_symbol": "ADORA2A",
  "term_label": "G protein-coupled adenosine receptor activity",
  "gene": "UniProtKB:P29274",
  "gene_name": "Adenosine receptor A2a"
}